{
  "term_id": "GO:0000122",
  "term_label": "negative regulation of transcription by RNA polymerase II",
  "gene_symbol": "LYAR",
  "gene_name": "Cell growth-regulating nucleolar protein",
  "gene": "UniProtKB:Q9NX58"
}